{
  "term_id": "GO:0000981",
  "gene_name": "Zinc finger and BTB domain-containing protein 38",
  "gene": "UniProtKB:Q8NAP3",
  "gene_symbol": "ZBTB38",
  "term_label": "DNA-binding transcription factor activity, RNA polymerase II-specific"
}